{
  "term_id": "UNKNOWN:0001",
  "gene_name": "Transmembrane emp24 domain-containing protein 4",
  "gene": "UniProtKB:Q7Z7H5",
  "gene_symbol": "TMED4",
  "term_label": "Unknown molecular function"
}